{
  "term_id": "GO:0005634",
  "gene": "UniProtKB:Q9H0Z9",
  "gene_name": "RNA-binding protein 38",
  "gene_symbol": "RBM38",
  "term_label": "nucleus"
}